{
  "term_label": "nucleus",
  "term_id": "GO:0005634",
  "gene": "UniProtKB:Q6ZN30",
  "gene_symbol": "BNC2",
  "gene_name": "Zinc finger protein basonuclin-2"
}